proline salvage [GO:0019492] (biological process) Also known as: proline cycling Sources: GOC:jl Definition: Any process which produces the amino acid proline from derivatives of it, without de novo synthesis. Relationships: is a type of amino acid salvage [GO:0043102]; is a type of GO:0055129